L-arabinose catabolic process [GO:0019572] (biological process) Sources: GOC:jsg, GOC:mah Relationships: is_a arabinose catabolic process [GO:0019568]; is a type of L-arabinose metabolic process [GO:0046373] Definition: The chemical reactions and pathways resulting in the breakdown of L-arabinose, the L-enantiomer of arabino-pentose. Subtypes: L-arabinose catabolic process to D-xylulose 5-phosphate [GO:0019569], L-arabinose catabolic process to 2-oxoglutarate [GO:0019570] Also known as: L-arabinose breakdown, L-arabinose catabolism, L-arabinose degradation